{
  "term_id": "GO:0006357",
  "gene_symbol": "MYF6",
  "gene_name": "Myogenic factor 6",
  "gene": "UniProtKB:P23409",
  "term_label": "regulation of transcription by RNA polymerase II"
}